{
  "term_label": "regulation of signal transduction",
  "term_id": "GO:0009966",
  "gene_symbol": "NCOA5",
  "gene": "UniProtKB:Q9HCD5",
  "gene_name": "Nuclear receptor coactivator 5"
}